natural killer cell proliferation [GO:0001787] (BP) Subtypes: GO:0002324 Regulation: regulated by GO:0032817; negatively regulated by negative regulation of natural killer cell proliferation [GO:0032818]; positively regulated by positive regulation of natural killer cell proliferation [GO:0032819] Definition: The expansion of a natural killer cell population by cell division. Relationships: is a type of natural killer cell activation [GO:0030101]; is a type of lymphocyte proliferation [GO:0046651] Also known as: NK cell proliferation Sources: GOC:add, ISBN:0781735149